subpallium cell migration [GO:0021980] (biological process) Subtypes: subpallium radially oriented migration [GO:0021981] Relationships: is a type of GO:0022029; is part of GO:0021544 Sources: GOC:cls, GOC:dgh, GOC:dph, GOC:jid, GO_REF:0000021 Definition: The orderly movement of cells from one site to another in the subpallium.